{
  "term_label": "Unknown molecular function",
  "gene": "UniProtKB:P58511",
  "gene_symbol": "SMIM11",
  "term_id": "UNKNOWN:0001",
  "gene_name": "Small integral membrane protein 11"
}